{
  "term_id": "UNKNOWN:0003",
  "gene_name": "Ankyrin repeat and SOCS box protein 15",
  "gene_symbol": "ASB15",
  "term_label": "Unknown cellular component",
  "gene": "UniProtKB:Q8WXK1"
}